peroxisome-mitochondrion membrane tether activity [GO:0160190] (molecular function) Definition: The binding activity of a molecule that brings together the peroxisome and the mitochondrial outer membrane, establishing the localization of the peroxisome close to the mitochondrion. References: PMID:29720625, PMID:38669296 Relationships: is a type of protein-membrane adaptor activity [GO:0043495]